dUTP catabolic process [GO:0046081] (biological process) Also known as: dUTP breakdown, dUTP catabolism, dUTP degradation Relationships: is a type of pyrimidine deoxyribonucleoside triphosphate catabolic process [GO:0009213]; is_a GO:0009223; is a type of dUTP metabolic process [GO:0046080] Definition: The chemical reactions and pathways resulting in the breakdown of dUTP, deoxyuridine (5'-)triphosphate. Sources: GOC:go_curators